N-terminal peptidyl-glycine methylation [GO:0018013] (biological process) Sources: RESID:AA0063 Definition: The methylation of the N-terminal glycine of proteins to form the derivative N-methylglycine. Relationships: is_a N-terminal protein amino acid methylation [GO:0006480]; is a type of peptidyl-glycine modification [GO:0018201]